{
  "gene": "UniProtKB:Q96QU1",
  "gene_name": "Protocadherin-15",
  "term_label": "photoreceptor outer segment",
  "gene_symbol": "PCDH15",
  "term_id": "GO:0001750"
}